{
  "gene_name": "Pleckstrin homology domain-containing family G member 1",
  "term_label": "Unknown biological process",
  "gene_symbol": "PLEKHG1",
  "gene": "UniProtKB:Q9ULL1",
  "term_id": "UNKNOWN:0002"
}